glyoxylate oxidase activity [GO:0047969] (molecular function) Sources: RHEA:14837 Relationships: is a type of oxidoreductase activity, acting on the aldehyde or oxo group of donors, oxygen as acceptor [GO:0016623] Definition: Catalysis of the reaction: glyoxylate + H2O + O2 = H2O2 + H+ + oxalate. Also known as: glyoxylate:oxygen oxidoreductase activity